{
  "term_id": "GO:0000082",
  "term_label": "G1/S transition of mitotic cell cycle",
  "gene_symbol": "CCNI",
  "gene": "UniProtKB:Q14094",
  "gene_name": "Cyclin-I"
}